{
  "term_label": "Unknown molecular function",
  "gene_name": "ADP-ribosylation factor-like protein 13A",
  "gene": "UniProtKB:Q5H913",
  "gene_symbol": "ARL13A",
  "term_id": "UNKNOWN:0001"
}